{
  "term_label": "endoplasmic reticulum",
  "gene_name": "3-hydroxy-3-methylglutaryl-CoA lyase, cytoplasmic",
  "gene_symbol": "HMGCLL1",
  "gene": "UniProtKB:Q8TB92",
  "term_id": "GO:0005783"
}